{
  "gene_symbol": "ZNF81",
  "gene_name": "Zinc finger protein 81",
  "gene": "UniProtKB:P51508",
  "term_label": "RNA polymerase II cis-regulatory region sequence-specific DNA binding",
  "term_id": "GO:0000978"
}